{
  "term_label": "synapse",
  "gene_symbol": "CALB1",
  "gene": "UniProtKB:P05937",
  "gene_name": "Calbindin",
  "term_id": "GO:0045202"
}